{
  "term_label": "phenylethanolamine N-methyltransferase activity",
  "gene_symbol": "PNMT",
  "gene_name": "Phenylethanolamine N-methyltransferase",
  "gene": "UniProtKB:P11086",
  "term_id": "GO:0004603"
}